positive regulation of cellular response to drug [GO:2001040] (biological process) Definition: Any process that activates or increases the frequency, rate or extent of cellular response to drug. Sources: GOC:obol Relationships: is a type of positive regulation of cellular process [GO:0048522]; is a type of positive regulation of response to drug [GO:2001025]; is a type of GO:2001038; positively regulates cellular response to xenobiotic stimulus [GO:0071466]